{
  "term_id": "GO:0005886",
  "term_label": "plasma membrane",
  "gene": "UniProtKB:Q86VH5",
  "gene_symbol": "LRRTM3",
  "gene_name": "Leucine-rich repeat transmembrane neuronal protein 3"
}